pulmonary artery endothelial tube morphogenesis [GO:0061155] (biological process) Sources: GOC:dph, GOC:yaf Definition: The process in which the anatomical structures of a tube are generated and organized from the pulmonary artery endothelium. An pulmonary artery endothelium is an epithelium that lines the pulmonary artery. Relationships: is a type of endothelial tube morphogenesis [GO:0061154]; is part of pulmonary artery morphogenesis [GO:0061156]